prophage integrase activity [GO:0008979] (molecular function) Also known as: integrase activity involved in establishment of integrated proviral latency Relationships: is a type of site-specific recombinase activity [GO:0009009]; is part of GO:0075713 Definition: Catalysis of the integration of prophage DNA into a target DNA molecule, usually a bacterial chromosome, via a sequence-specific recombination event which involves the formation of an intasome, a DNA-protein-complex designed for site-specific recombination of the phage and host DNA. Sources: GOC:jl